malonate(1-) transmembrane transporter activity [GO:1901239] (molecular function) References: PMID:9128730, PMID:9573154 Sources: GOC:TermGenie Also known as: malonic acid uptake transmembrane transporter activity Definition: Enables the transfer of malonate(1-) from one side of a membrane to the other. Subtypes: GO:0044668 Relationships: is a type of dicarboxylic acid transmembrane transporter activity [GO:0005310]; BFO_0000050 GO:1901553